{
  "gene_name": "Alpha-sarcoglycan",
  "term_label": "sarcoglycan complex",
  "gene_symbol": "SGCA",
  "gene": "UniProtKB:Q16586",
  "term_id": "GO:0016012"
}